{
  "gene_name": "Spermidine synthase",
  "term_label": "spermidine biosynthetic process",
  "term_id": "GO:0008295",
  "gene_symbol": "SRM",
  "gene": "UniProtKB:P19623"
}